proton motive force-driven plasma membrane ATP synthesis [GO:0042777] (biological process) Also known as: ATP synthesis coupled proton transport, plasma membrane ATP synthesis coupled proton transport Definition: The chemical reactions and pathways resulting in the formation of ATP driven by transport of protons across a plasma membrane to generate an electrochemical gradient (proton-motive force). Relationships: is a type of proton motive force-driven ATP synthesis [GO:0015986] Sources: GOC:vw